pancreatic PP cell fate commitment [GO:0003329] (BP) Definition: The commitment of a cell to a pancreatic PP cell fate and its capacity to differentiate into a pancreatic PP cell. A pancreatic polypeptide-producing cell is a cell in the pancreas that produces pancreatic polypeptide. Relationships: is a type of epithelial cell fate commitment [GO:0072148]; is part of GO:0003312 Sources: GOC:dph